atrial septum primum morphogenesis [GO:0003289] (biological process) Definition: The process in which anatomical structure of an atrial septum primum is generated and organized. Sources: GOC:mtg_heart Relationships: is a type of GO:0060413; is part of septum primum development [GO:0003284]